tyrocidine catabolic process [GO:1901903] (biological process) Definition: The chemical reactions and pathways resulting in the breakdown of tyrocidine. References: PMID:9352938 Sources: GOC:TermGenie, GOC:yaf Also known as: tyrocidine breakdown, tyrocidine catabolism, tyrocidine degradation Relationships: is a type of catabolic process [GO:0009056]